proximal stomach smooth muscle contraction [GO:0014847] (biological process) Relationships: is a type of tonic smooth muscle contraction [GO:0014820]; is a type of stomach smooth muscle contraction [GO:0120063] References: PMID:30252381 Sources: GOC:mtg_muscle Definition: A process in which force is generated within smooth muscle tissue, resulting in a change in muscle geometry. This process occurs in the proximal stomach. Force generation involves a chemo-mechanical energy conversion step that is carried out by the actin/myosin complex activity, which generates force through ATP hydrolysis. The proximal stomach, composed of the fundus and upper body, shows low frequency, sustained tonic contractions that are responsible for generating a basal pressure within the stomach. Subtypes: stomach fundus smooth muscle contraction [GO:0014825]